{
  "term_id": "GO:0005739",
  "gene": "UniProtKB:O15079",
  "term_label": "mitochondrion",
  "gene_symbol": "SNPH",
  "gene_name": "Syntaphilin"
}